succinyl-CoA metabolic process [GO:0006104] (biological process) Relationships: is_a acyl-CoA metabolic process [GO:0006637] Subtypes: GO:0006781, L-methionine catabolic process to succinyl-CoA [GO:0019457], tetrapyrrole biosynthetic process from glycine and succinyl-CoA [GO:0033527], succinyl-CoA catabolic process [GO:1901289], succinyl-CoA biosynthetic process [GO:1901290] Also known as: succinyl-CoA metabolism Definition: The chemical reactions and pathways involving succinyl-CoA, a compound composed of the monovalent acyl group 3-carboxypropanoyl, derived from succinic acid by loss of one OH group, linked to coenzyme A. Sources: GOC:ai